{
  "gene": "UniProtKB:Q8WVT3",
  "term_id": "UNKNOWN:0002",
  "term_label": "Unknown biological process",
  "gene_symbol": "TRAPPC12",
  "gene_name": "Trafficking protein particle complex subunit 12"
}